{
  "term_id": "UNKNOWN:0001",
  "gene": "UniProtKB:Q9BWG6",
  "gene_name": "Sodium channel modifier 1",
  "term_label": "Unknown molecular function",
  "gene_symbol": "SCNM1"
}